{
  "gene_symbol": "ABCD3",
  "term_id": "GO:0015910",
  "term_label": "long-chain fatty acid import into peroxisome",
  "gene_name": "ATP-binding cassette sub-family D member 3",
  "gene": "UniProtKB:P28288"
}